{
  "gene_symbol": "OR52J3",
  "term_id": "GO:0004984",
  "term_label": "olfactory receptor activity",
  "gene": "UniProtKB:Q8NH60",
  "gene_name": "Olfactory receptor 52J3"
}